{
  "term_label": "DNA-binding transcription factor activity, RNA polymerase II-specific",
  "term_id": "GO:0000981",
  "gene": "UniProtKB:Q92826",
  "gene_name": "Homeobox protein Hox-B13",
  "gene_symbol": "HOXB13"
}